{
  "term_id": "GO:0055070",
  "gene_name": "COMM domain-containing protein 1",
  "gene_symbol": "COMMD1",
  "gene": "UniProtKB:Q8N668",
  "term_label": "copper ion homeostasis"
}